{
  "gene_name": "Adenylosuccinate lyase",
  "gene": "UniProtKB:P30566",
  "term_label": "(S)-2-(5-amino-1-(5-phospho-D-ribosyl)imidazole-4-carboxamido) succinate lyase (fumarate-forming) activity",
  "term_id": "GO:0070626",
  "gene_symbol": "ADSL"
}